high-affinity copper ion transmembrane transporter activity [GO:0015089] (molecular function) Relationships: is a type of copper ion transmembrane transporter activity [GO:0005375] Definition: Enables the transfer of a copper ions (Cu2+) from one side of a membrane to the other. In high-affinity transport the transporter is able to bind the solute even if it is only present at very low concentrations. Also known as: high affinity copper ion transmembrane transporter activity, high affinity copper transporter activity Sources: TC:9.A.11.1.1